isoflavonoid biosynthetic process [GO:0009717] (biological process) Sources: GOC:ai Also known as: isoflavonoid anabolism, isoflavonoid biosynthesis, isoflavonoid formation, isoflavonoid synthesis Definition: The chemical reactions and pathways resulting in the formation of isoflavonoids, a group of water-soluble phenolic derivatives, isomeric with flavonoids. Subtypes: isoflavonoid phytoalexin biosynthetic process [GO:0009701] Relationships: is_a phenylpropanoid biosynthetic process [GO:0009699]; is_a GO:0046287